{
  "gene_symbol": "ANKRD36B",
  "gene_name": "Ankyrin repeat domain-containing protein 36B",
  "term_label": "Unknown molecular function",
  "term_id": "UNKNOWN:0001",
  "gene": "UniProtKB:Q8N2N9"
}